{
  "gene_symbol": "PGP",
  "gene_name": "Glycerol-3-phosphate phosphatase",
  "term_id": "GO:0043136",
  "gene": "UniProtKB:A6NDG6",
  "term_label": "sn-glycerol 3-phosphatase activity"
}